{
  "term_id": "UNKNOWN:0001",
  "term_label": "Unknown molecular function",
  "gene": "UniProtKB:Q5U649",
  "gene_name": "Uncharacterized protein C12orf60",
  "gene_symbol": "C12orf60"
}